negative regulation of neuronal signal transduction [GO:1902848] (biological process) Definition: Any process that stops, prevents or reduces the frequency, rate or extent of neuronal signal transduction. Sources: GOC:TermGenie, GOC:sjp, GO_REF:0000058 Relationships: is_a negative regulation of signal transduction [GO:0009968]; is a type of regulation of neuronal signal transduction [GO:1902847]; negatively regulates neuronal signal transduction [GO:0023041] Also known as: down regulation of neuronal signal transduction, down-regulation of neuronal signal transduction, downregulation of neuronal signal transduction, inhibition of neuronal signal transduction